{
  "gene_name": "RISC-loading complex subunit TARBP2",
  "gene_symbol": "TARBP2",
  "term_label": "nucleus",
  "term_id": "GO:0005634",
  "gene": "UniProtKB:Q15633"
}